G protein-coupled glutamate receptor activity [GO:0098988] (molecular function) Definition: Combining with glutamate and transmitting a signal from one side of the membrane to the other by activating an associated G-protein, initiating a change in cell activity. Relationships: is a type of G protein-coupled receptor activity [GO:0004930]; is a type of GO:0008066 Subtypes: GO:0001639, GO:0001640 Also known as: G-protein coupled glutamate receptor activity Sources: GOC:dos